{
  "gene_symbol": "BMP7",
  "term_label": "heart development",
  "gene_name": "Bone morphogenetic protein 7",
  "term_id": "GO:0007507",
  "gene": "UniProtKB:P18075"
}